{
  "gene_name": "Olfactory receptor 11G2",
  "gene_symbol": "OR11G2",
  "term_label": "Unknown molecular function",
  "gene": "UniProtKB:Q8NGC1",
  "term_id": "UNKNOWN:0001"
}